{
  "term_label": "DNA damage response",
  "gene": "UniProtKB:Q5MIZ7",
  "term_id": "GO:0006974",
  "gene_symbol": "PPP4R3B",
  "gene_name": "Serine_threonine-protein phosphatase 4 regulatory subunit 3B"
}